elongin complex [GO:0070449] (cellular component) Relationships: is a type of GO:0008023 Definition: A transcription elongation factor complex that suppresses RNA polymerase II pausing, and may act by promoting proper alignment of the 3'-end of nascent transcripts with the polymerase catalytic site. Consists of a transcriptionally active Elongin A subunit (about 100 kDa) and two smaller Elongin B (about 18 kDa) and Elongin C (about 15 kDa) subunits. Note: See also the cellular component terms 'cyclin-dependent protein kinase activating kinase holoenzyme complex ; GO:0019907' and 'DNA-directed RNA polymerase II, holoenzyme ; GO:0016591'. References: PMID:12676794 Also known as: elongin (SIII) complex, transcription elongation factor SIII complex, transcription factor B (SIII) complex